negative regulation of proteolysis [GO:0045861] (biological process) Sources: GOC:go_curators Also known as: down regulation of proteolysis, down-regulation of proteolysis, downregulation of proteolysis, negative regulation of peptidolysis, inhibition of proteolysis Relationships: is a type of regulation of proteolysis [GO:0030162]; is a type of negative regulation of protein metabolic process [GO:0051248]; negatively regulates GO:0006508 Definition: Any process that stops, prevents, or reduces the frequency, rate or extent of the hydrolysis of a peptide bond or bonds within a protein. Subtypes: negative regulation of peptidase activity [GO:0010466], negative regulation of protein processing [GO:0010955], GO:0051045, negative regulation of proteolysis involved in protein catabolic process [GO:1903051]